{
  "gene": "UniProtKB:Q8TD10",
  "term_id": "UNKNOWN:0002",
  "gene_name": "Mirror-image polydactyly gene 1 protein",
  "gene_symbol": "MIPOL1",
  "term_label": "Unknown biological process"
}